{
  "term_id": "UNKNOWN:0002",
  "gene": "UniProtKB:P21333",
  "gene_name": "Filamin-A",
  "gene_symbol": "FLNA",
  "term_label": "Unknown biological process"
}